{
  "gene": "UniProtKB:Q92540",
  "gene_symbol": "SMG7",
  "term_label": "telomerase holoenzyme complex",
  "gene_name": "Nonsense-mediated mRNA decay factor SMG7",
  "term_id": "GO:0005697"
}